{
  "term_id": "UNKNOWN:0001",
  "gene_symbol": "A0A8I5KYW3",
  "gene": "UniProtKB:A0A8I5KYW3",
  "term_label": "Unknown molecular function",
  "gene_name": "Uncharacterized protein"
}